{
  "gene_symbol": "CUL4A",
  "term_id": "GO:0043161",
  "gene": "UniProtKB:Q13619",
  "term_label": "proteasome-mediated ubiquitin-dependent protein catabolic process",
  "gene_name": "Cullin-4A"
}